respiratory chain complex II (succinate dehydrogenase) [GO:0045273] (cellular component) Also known as: electron transport complex II Relationships: is a type of membrane protein complex [GO:0098796]; is_a respiratory chain complex [GO:0098803]; is a type of GO:1990204 Sources: ISBN:0198547684 Definition: A part of the respiratory chain, containing the four polypeptide subunits of succinate dehydrogenase, flavin-adenine dinucleotide and iron-sulfur. Catalyzes the oxidation of succinate by ubiquinone. Connects the TCA cycle with the respiratory chain.